{
  "term_label": "Wnt-protein binding",
  "gene_name": "Secreted frizzled-related protein 5",
  "gene": "UniProtKB:Q5T4F7",
  "term_id": "GO:0017147",
  "gene_symbol": "SFRP5"
}